{
  "gene_symbol": "RANBP10",
  "gene_name": "Ran-binding protein 10",
  "term_id": "GO:0043161",
  "term_label": "proteasome-mediated ubiquitin-dependent protein catabolic process",
  "gene": "UniProtKB:Q6VN20"
}